{
  "gene_name": "Transmembrane protein C16orf54",
  "gene": "UniProtKB:Q6UWD8",
  "term_id": "UNKNOWN:0002",
  "term_label": "Unknown biological process",
  "gene_symbol": "C16orf54"
}